skeletal muscle satellite cell commitment [GO:0014813] (BP) Relationships: is a type of cell fate commitment [GO:0045165]; BFO_0000050 skeletal muscle satellite cell differentiation [GO:0014816] Definition: The process in which the developmental fate of a cell becomes restricted such that it will develop into a satellite cell. References: PMID:16607119 Sources: GOC:ef, GOC:mtg_muscle